DNA bending complex [GO:1990104] (cellular component) References: PMID:17097674 Sources: GOC:bhm Also known as: histone-like DNA binding complex Definition: A protein-DNA complex that contains DNA in combination with a protein which binds to and bends DNA. Often plays a role in DNA compaction. Relationships: is a type of protein-containing complex [GO:0032991] Subtypes: GO:1990121, IHF-DNA complex [GO:1990177], HU-DNA complex [GO:1990178]